{
  "gene_name": "Tumor protein p73",
  "gene_symbol": "TP73",
  "term_label": "RNA polymerase II cis-regulatory region sequence-specific DNA binding",
  "term_id": "GO:0000978",
  "gene": "UniProtKB:O15350"
}